{
  "gene_name": "SHC-transforming protein 1",
  "gene": "UniProtKB:P29353",
  "term_label": "epidermal growth factor receptor signaling pathway",
  "term_id": "GO:0007173",
  "gene_symbol": "SHC1"
}